{
  "gene_name": "TNF receptor-associated factor 5",
  "gene": "UniProtKB:O00463",
  "term_label": "signaling adaptor activity",
  "gene_symbol": "TRAF5",
  "term_id": "GO:0035591"
}